NEDD8 ligase activity [GO:0061663] (molecular function) Sources: GOC:dph Definition: Catalysis of the transfer of NEDD8 to a substrate protein via the reaction X-NEDD8 + S = X + S-NEDD8, where X is either an E2 or E3 enzyme, the X-NEDD8 linkage is a thioester bond, and the S-NEDD8 linkage is an isopeptide bond between the C-terminal amino acid of NEDD8 and the epsilon-amino group of lysine residues in the substrate. Relationships: is a type of NEDD8 transferase activity [GO:0019788]; is_a GO:0061659 Also known as: E3